{
  "gene_symbol": "HMX3",
  "gene": "UniProtKB:A6NHT5",
  "term_label": "DNA-binding transcription factor activity, RNA polymerase II-specific",
  "gene_name": "Homeobox protein HMX3",
  "term_id": "GO:0000981"
}